regulation of vesicle docking [GO:0106020] (biological process) Relationships: is a type of regulation of localization [GO:0032879]; is a type of GO:0050794; regulates vesicle docking [GO:0048278] Also known as: regulation of vesicle to membrane docking Definition: Any process that modulates the frequency, rate or extent of vesicle docking. References: PMID:22810233 Subtypes: regulation of exocyst assembly [GO:0001928], GO:0099148, negative regulation of vesicle docking [GO:0106021], positive regulation of vesicle docking [GO:0106022]